{
  "term_label": "Unknown molecular function",
  "gene_name": "m7GpppN-mRNA hydrolase",
  "gene_symbol": "DCP2",
  "term_id": "UNKNOWN:0001",
  "gene": "UniProtKB:Q8IU60"
}